{
  "gene": "UniProtKB:Q86TM3",
  "term_id": "UNKNOWN:0003",
  "gene_symbol": "DDX53",
  "term_label": "Unknown cellular component",
  "gene_name": "Probable ATP-dependent RNA helicase DDX53"
}